{
  "term_label": "neutral L-amino acid transmembrane transporter activity",
  "gene_name": "Excitatory amino acid transporter 4",
  "term_id": "GO:0015175",
  "gene_symbol": "SLC1A6",
  "gene": "UniProtKB:P48664"
}